anaphase-promoting complex [GO:0005680] (cellular component) Relationships: is_a GO:0000152; is a type of cullin-RING ubiquitin ligase complex [GO:0031461] References: PMID:10465783, PMID:10611969 Sources: GOC:jh, GOC:vw Note: Note that the synonym 'APC' should not be confused with the abbreviation for the adenomatous polyposis coli gene and protein. Also known as: APC, anaphase promoting complex, cyclosome Definition: A ubiquitin ligase complex that degrades mitotic cyclins and anaphase inhibitory protein, thereby triggering sister chromatid separation and exit from mitosis. Substrate recognition by APC occurs through degradation signals, the most common of which is termed the Dbox degradation motif, originally discovered in cyclin B.